{
  "gene_name": "Olfactory receptor 4C16",
  "term_label": "Unknown biological process",
  "term_id": "UNKNOWN:0002",
  "gene": "UniProtKB:Q8NGL9",
  "gene_symbol": "OR4C16"
}